{
  "gene_symbol": "RPL36A",
  "term_id": "GO:0003735",
  "gene": "UniProtKB:P83881",
  "gene_name": "Large ribosomal subunit protein eL42",
  "term_label": "structural constituent of ribosome"
}